{
  "gene": "UniProtKB:O75084",
  "term_label": "canonical Wnt signaling pathway",
  "gene_symbol": "FZD7",
  "gene_name": "Frizzled-7",
  "term_id": "GO:0060070"
}